{
  "gene_symbol": "TMEM209",
  "term_label": "membrane",
  "term_id": "GO:0016020",
  "gene": "UniProtKB:Q96SK2",
  "gene_name": "Transmembrane protein 209"
}